negative regulation of SCF-dependent proteasomal ubiquitin-dependent catabolic process [GO:0062026] (biological process) Relationships: is a type of negative regulation of proteasomal ubiquitin-dependent protein catabolic process [GO:0032435]; is a type of GO:0062025; negatively regulates SCF-dependent proteasomal ubiquitin-dependent protein catabolic process [GO:0031146] References: PMID:28007894 Definition: Any process that stops or decreases the rate, frequency or extent of SCF-dependent proteasomal ubiquitin-dependent protein catabolic process, the chemical reactions and pathways resulting in the breakdown of a protein or peptide by hydrolysis of its peptide bonds, initiated by the covalent attachment of ubiquitin, with ubiquitin-protein ligation catalyzed by an SCF (Skp1/Cul1/F-box protein) complex, and mediated by the proteasome.